{
  "term_label": "TRAMP complex",
  "gene": "UniProtKB:Q5XG87",
  "term_id": "GO:0031499",
  "gene_symbol": "TENT4A",
  "gene_name": "Terminal nucleotidyltransferase 4A"
}